{
  "gene": "UniProtKB:Q9BZS1",
  "gene_name": "Forkhead box protein P3",
  "term_id": "GO:0006357",
  "gene_symbol": "FOXP3",
  "term_label": "regulation of transcription by RNA polymerase II"
}